{
  "term_label": "DNA-binding transcription factor activity, RNA polymerase II-specific",
  "gene": "UniProtKB:A0AVK6",
  "gene_name": "Transcription factor E2F8",
  "term_id": "GO:0000981",
  "gene_symbol": "E2F8"
}